{
  "gene_name": "Prostaglandin reductase 2",
  "gene_symbol": "PTGR2",
  "term_label": "prostaglandin metabolic process",
  "term_id": "GO:0006693",
  "gene": "UniProtKB:Q8N8N7"
}